{
  "gene_name": "Immunity-related GTPase family M protein",
  "gene_symbol": "IRGM",
  "term_id": "GO:0035458",
  "gene": "UniProtKB:A1A4Y4",
  "term_label": "cellular response to interferon-beta"
}